regulation of clathrin coat assembly [GO:1905443] (biological process) Subtypes: negative regulation of clathrin coat assembly [GO:1905444], positive regulation of clathrin coat assembly [GO:1905445] Also known as: regulation of clathrin cage assembly References: PMID:15533940 Sources: GOC:PARL, GOC:TermGenie, GOC:bf, GO_REF:0000058 Relationships: is_a regulation of protein-containing complex assembly [GO:0043254]; regulates clathrin coat assembly [GO:0048268] Definition: Any process that modulates the frequency, rate or extent of clathrin coat assembly.